gravitropism [GO:0009630] (biological process) Relationships: is a type of tropism [GO:0009606]; is a type of response to gravity [GO:0009629] Subtypes: GO:0009958, negative gravitropism [GO:0009959] Definition: The orientation of plant parts under the stimulation of gravity. Sources: ISBN:0198547684 Also known as: geotropism